calcitonin secretion [GO:0036161] (biological process) Relationships: is a type of peptide hormone secretion [GO:0030072] Regulation: regulated by regulation of calcitonin secretion [GO:1904362]; negatively regulated by negative regulation of calcitonin secretion [GO:1904363]; positively regulated by GO:1904364 Definition: The regulated release of calcitonin, a peptide hormone that participates in calcium and phosphorus metabolism, from a cell. Sources: GOC:cjm